{
  "gene": "UniProtKB:Q9HD67",
  "gene_name": "Unconventional myosin-X",
  "term_id": "GO:0051015",
  "gene_symbol": "MYO10",
  "term_label": "actin filament binding"
}